Nebenkern [GO:0016006] (cellular component) Definition: A product of the fusion of the mitochondria during spermatogenesis. After the completion of meiosis the mitochondria of the spermatid collect along side the nucleus and fuse into two masses; these wrap around each other to produce the spherical Nebenkern. During flagellum elongation the Nebenkern unfolds and the two derivatives (major and minor mitochondrial derivatives) elongate down the axoneme. References: PMID:25265054 Sources: GOC:ma Relationships: is a type of mitochondrial derivative [GO:0016007]